germarium-derived female germ-line cyst formation [GO:0030727] (biological process) Also known as: germarium-derived female germline cyst formation Relationships: is a type of female germ-line cyst formation [GO:0048135]; is part of germarium-derived egg chamber formation [GO:0007293] References: PMID:10370240, PMID:9442902 Sources: GOC:mtg_sensu Definition: Formation, in a germarium, of a group of interconnected cells derived from a single female gonial founder cell (a cystoblast). The germarium is the most anterior portion of an insect ovariole. An example of this process is found in Drosophila melanogaster.